{
  "term_id": "UNKNOWN:0001",
  "gene_name": "Nucleolar protein 11",
  "gene": "UniProtKB:Q9H8H0",
  "gene_symbol": "NOL11",
  "term_label": "Unknown molecular function"
}